{
  "gene": "UniProtKB:Q8N5Y8",
  "term_id": "GO:0019900",
  "gene_symbol": "PARP16",
  "term_label": "kinase binding",
  "gene_name": "Protein mono-ADP-ribosyltransferase PARP16"
}